{
  "term_label": "extracellular region",
  "term_id": "GO:0005576",
  "gene_symbol": "CHIT1",
  "gene_name": "Chitotriosidase-1",
  "gene": "UniProtKB:Q13231"
}